{
  "gene_symbol": "FYN",
  "gene_name": "Tyrosine-protein kinase Fyn",
  "term_label": "cell differentiation",
  "gene": "UniProtKB:P06241",
  "term_id": "GO:0030154"
}